{
  "gene": "UniProtKB:A0A7P0TBJ1",
  "gene_symbol": "HAPSTR2",
  "gene_name": "HUWE1-associated protein modifying stress responses 2",
  "term_label": "Unknown biological process",
  "term_id": "UNKNOWN:0002"
}